rRNA (guanine-N2-)-methyltransferase activity [GO:0008990] (molecular function) Relationships: is a type of N-methyltransferase activity [GO:0008170]; is a type of rRNA (guanine) methyltransferase activity [GO:0016435] Also known as: S-adenosyl-L-methionine:rRNA (guanine-2-N-)-methyltransferase activity, S-adenosyl-L-methionine:rRNA (guanine-N2-)-methyltransferase activity, ribosomal ribonucleate guanine-2-methyltransferase activity Subtypes: 16S rRNA (guanine(1516)-N(2))-methyltransferase activity [GO:0036308], 16S rRNA (guanine(966)-N(2))-methyltransferase activity [GO:0052913], GO:0052914, 23S rRNA (guanine(2445)-N(2))-methyltransferase activity [GO:0052915], 23S rRNA (guanine(1835)-N(2))-methyltransferase activity [GO:0052916] Definition: Catalysis of the reaction: S-adenosyl-L-methionine + rRNA = S-adenosyl-L-homocysteine + rRNA containing N2-methylguanine. References: PMID:17389639